symbiont-mediated hemolysis of host erythrocyte [GO:0019836] (biological process) Relationships: is_a symbiont-mediated cytolysis of host cell [GO:0001897] Sources: GOC:add, UniProtKB-KW:KW-0354 Also known as: pathogenesis, haemolysis in host, hemolysis by symbiont of host RBCs, hemolysis by symbiont of host erythrocytes, hemolysis by symbiont of host red blood cells, regulation of cytolysis of host cells by symbiont, hemolysin activity Definition: The cytolytic destruction of red blood cells, with the release of intracellular hemoglobin, in the host organism by a symbiont. The host is defined as the larger of the organisms involved in a symbiotic interaction.